{
  "gene_symbol": "TMED7",
  "gene_name": "Transmembrane emp24 domain-containing protein 7",
  "gene": "UniProtKB:Q9Y3B3",
  "term_label": "endoplasmic reticulum-Golgi intermediate compartment",
  "term_id": "GO:0005793"
}